{
  "gene_symbol": "TNFRSF21",
  "term_id": "GO:0005886",
  "gene_name": "Tumor necrosis factor receptor superfamily member 21",
  "gene": "UniProtKB:O75509",
  "term_label": "plasma membrane"
}